negative regulation of CD4-positive, alpha-beta T cell proliferation [GO:2000562] (biological process) Sources: GOC:obol Relationships: is a type of negative regulation of alpha-beta T cell proliferation [GO:0046642]; is a type of negative regulation of CD4-positive, alpha-beta T cell activation [GO:2000515]; is a type of regulation of CD4-positive, alpha-beta T cell proliferation [GO:2000561]; negatively regulates CD4-positive, alpha-beta T cell proliferation [GO:0035739] Definition: Any process that stops, prevents or reduces the frequency, rate or extent of CD4-positive, alpha-beta T cell proliferation.